negative regulation of pre-B cell receptor expression [GO:0140646] (BP) References: PMID:22949502 Relationships: is a type of negative regulation of cellular process [GO:0048523]; is a type of GO:0051093; negatively regulates pre-B cell receptor expression [GO:0002330] Definition: Any process that stops, prevents or reduces the frequency, rate or extent of the process leading up to expression of the pre-B cell receptor on the surface of pre-B cells.